{
  "gene_name": "Calnexin",
  "gene_symbol": "CANX",
  "term_label": "endoplasmic reticulum membrane",
  "gene": "UniProtKB:P27824",
  "term_id": "GO:0005789"
}